leukotriene D4 biosynthetic process [GO:1901750] (biological process) Relationships: is a type of leukotriene biosynthetic process [GO:0019370]; is a type of amide biosynthetic process [GO:0043604]; is_a sulfur compound biosynthetic process [GO:0044272]; is a type of fatty acid derivative biosynthetic process [GO:1901570] Also known as: leukotriene D4 anabolism, leukotriene D4 biosynthesis, leukotriene D4 formation, leukotriene D4 synthesis Sources: GOC:TermGenie, GOC:yaf, UniPathway:UPA00880 Definition: The chemical reactions and pathways resulting in the formation of leukotriene D4.